{
  "gene_symbol": "ANGPT1",
  "term_id": "GO:0005615",
  "term_label": "extracellular space",
  "gene_name": "Angiopoietin-1",
  "gene": "UniProtKB:Q15389"
}